acetylcholine uptake [GO:0051630] (biological process) Definition: The directed movement of acetylcholine into a cell, typically presynaptic neurons or glial cells. Acetylcholine is a major neurotransmitter and neuromodulator both in the central and peripheral nervous systems. It also acts as a paracrine signal in various non-neural tissues. Regulation: regulated by regulation of acetylcholine uptake [GO:0051631]; negatively regulated by negative regulation of acetylcholine uptake [GO:0051632]; positively regulated by positive regulation of acetylcholine uptake [GO:0051633] Also known as: acetylcholine import Sources: GOC:ai Relationships: is a type of acetylcholine transport [GO:0015870]